{
  "gene_symbol": "GALNT15",
  "gene": "UniProtKB:Q8N3T1",
  "term_id": "GO:0004653",
  "term_label": "polypeptide N-acetylgalactosaminyltransferase activity",
  "gene_name": "Polypeptide N-acetylgalactosaminyltransferase 15"
}